basement membrane assembly involved in embryonic body morphogenesis [GO:2001197] (biological process) Relationships: is a type of cellular component assembly involved in morphogenesis [GO:0010927]; is a type of basement membrane assembly [GO:0070831]; is part of GO:0010172 Definition: Any basement membrane assembly that is involved in embryonic body morphogenesis. Sources: GOC:obol Regulation: regulated by regulation of basement membrane assembly involved in embryonic body morphogenesis [GO:1904259]; negatively regulated by negative regulation of basement membrane assembly involved in embryonic body morphogenesis [GO:1904260]; positively regulated by positive regulation of basement membrane assembly involved in embryonic body morphogenesis [GO:1904261]